{
  "term_label": "heparin binding",
  "gene": "UniProtKB:P58658",
  "gene_name": "Protein eva-1 homolog C",
  "term_id": "GO:0008201",
  "gene_symbol": "EVA1C"
}